{
  "term_label": "nucleus",
  "gene": "UniProtKB:A0A1W2PPD8",
  "term_id": "GO:0005634",
  "gene_symbol": "KDM4F",
  "gene_name": "Probable lysine-specific demethylase 4F"
}